{
  "gene_name": "Trans-acting T-cell-specific transcription factor GATA-3",
  "gene_symbol": "GATA3",
  "term_id": "GO:0048568",
  "gene": "UniProtKB:P23771",
  "term_label": "embryonic organ development"
}